B-1 B cell proliferation [GO:0002359] (BP) Sources: GOC:jal Also known as: B-1 B lymphocyte proliferation, B-1 B-cell proliferation, B-1 B-lymphocyte proliferation Relationships: is a type of B cell proliferation [GO:0042100] Definition: The expansion of a B-1 B cell by cell division. Follows B cell activation.